pexophagy [GO:0000425] (biological process) Definition: The selective autophagy process in which a peroxisome is degraded by macroautophagy. Also known as: macropexophagy Relationships: is a type of macroautophagy [GO:0016236]; is a type of GO:0030242 References: PMID:12914914, PMID:16973210 Sources: GOC:autophagy